{
  "gene_symbol": "SEMA5B",
  "gene_name": "Semaphorin-5B",
  "term_id": "GO:0030335",
  "gene": "UniProtKB:Q9P283",
  "term_label": "positive regulation of cell migration"
}